immune response in brain or nervous system [GO:0002383] (biological process) Relationships: is a type of organ or tissue specific immune response [GO:0002251] Sources: GOC:jal, GO_REF:0000022, ISBN:0781735149 Definition: An immune response taking place in the brain or nervous system.